{
  "gene_symbol": "TTC21A",
  "term_id": "GO:0035721",
  "gene_name": "Tetratricopeptide repeat protein 21A",
  "gene": "UniProtKB:Q8NDW8",
  "term_label": "intraciliary retrograde transport"
}